collagen biosynthetic process [GO:0032964] (biological process) Relationships: is a type of biosynthetic process [GO:0009058]; is a type of collagen metabolic process [GO:0032963] Also known as: collagen anabolism, collagen biosynthesis, collagen formation, collagen synthesis Sources: GOC:mah, ISBN:0198506732 Definition: The chemical reactions and pathways resulting in the formation of collagen, any of a group of fibrous proteins of very high tensile strength that form the main component of connective tissue in animals. Collagen is highly enriched in glycine (some regions are 33% glycine) and proline, occurring predominantly as 3-hydroxyproline (about 20%). Regulation: regulated by regulation of collagen biosynthetic process [GO:0032965]; negatively regulated by negative regulation of collagen biosynthetic process [GO:0032966]; positively regulated by positive regulation of collagen biosynthetic process [GO:0032967]